{
  "gene_name": "Dihydrolipoyllysine-residue acetyltransferase component of pyruvate dehydrogenase complex, mitochondrial",
  "gene": "UniProtKB:P10515",
  "term_id": "GO:0005739",
  "term_label": "mitochondrion",
  "gene_symbol": "DLAT"
}